{
  "gene": "UniProtKB:Q8NGJ0",
  "gene_symbol": "OR5A1",
  "term_label": "Unknown cellular component",
  "gene_name": "Olfactory receptor 5A1",
  "term_id": "UNKNOWN:0003"
}